{
  "gene": "UniProtKB:Q5T319",
  "term_label": "Unknown biological process",
  "gene_symbol": "FAM182B",
  "term_id": "UNKNOWN:0002",
  "gene_name": "Protein FAM182B"
}